{
  "gene_name": "Heme-binding protein 2",
  "gene": "UniProtKB:Q9Y5Z4",
  "term_label": "heme binding",
  "gene_symbol": "HEBP2",
  "term_id": "GO:0020037"
}